{
  "gene_symbol": "TARBP2",
  "gene": "UniProtKB:Q15633",
  "gene_name": "RISC-loading complex subunit TARBP2",
  "term_id": "GO:0003725",
  "term_label": "double-stranded RNA binding"
}